microtubule plus-end directed mitotic chromosome migration [GO:0099606] (biological process) Relationships: is a type of microtubule-based movement [GO:0007018]; is a type of chromosome localization [GO:0050000]; is a type of establishment of localization in cell [GO:0051649]; is a type of establishment of organelle localization [GO:0051656]; is a type of mitotic cell cycle process [GO:1903047]; is part of mitotic metaphase chromosome alignment [GO:0007080] References: PMID:26258632, PMID:26705896 Sources: GOC:dos Also known as: plus-end directed chromosome gliding Definition: The cell cycle process in which chromosomes that are laterally attached to one or more mitotic spindle microtubules migrate towards the spindle equator via plus-end-directed movement along the microtubules. This process is part of mitotic metaphase plate congression.